{
  "gene_name": "Msx2-interacting protein",
  "term_id": "GO:0006357",
  "term_label": "regulation of transcription by RNA polymerase II",
  "gene": "UniProtKB:Q96T58",
  "gene_symbol": "SPEN"
}